positive regulation of cilium beat frequency involved in ciliary motility [GO:0120030] (biological process) Relationships: is a type of regulation of cilium beat frequency involved in ciliary motility [GO:0060296] References: PMID:28035044 Definition: Any process that activates or increases the frequency of cilium beating involved in ciliary motility.